{
  "gene_symbol": "WDFY2",
  "gene_name": "WD repeat and FYVE domain-containing protein 2",
  "term_label": "Unknown molecular function",
  "term_id": "UNKNOWN:0001",
  "gene": "UniProtKB:Q96P53"
}